{
  "gene": "UniProtKB:Q7Z3S9",
  "term_label": "Unknown molecular function",
  "term_id": "UNKNOWN:0001",
  "gene_name": "Notch homolog 2 N-terminal-like protein A",
  "gene_symbol": "NOTCH2NLA"
}